gibberellin carboxyl-O-methyltransferase activity [GO:0010341] (molecular function) References: PMID:17220201 Definition: Catalysis of the reaction: S-adenosyl-L-methionine + a gibberellin = S-adenosyl-L-homocysteine + a gibberellin methyl ester. Relationships: is_a carboxyl-O-methyltransferase activity [GO:0010340]